{
  "gene_symbol": "RFLNB",
  "gene_name": "Refilin-B",
  "term_id": "GO:0061182",
  "term_label": "negative regulation of chondrocyte development",
  "gene": "UniProtKB:Q8N5W9"
}